{
  "gene_symbol": "EVI2B",
  "term_id": "UNKNOWN:0003",
  "gene": "UniProtKB:P34910",
  "gene_name": "Protein EVI2B",
  "term_label": "Unknown cellular component"
}